{
  "gene_symbol": "CXCL10",
  "term_label": "cellular response to lipopolysaccharide",
  "gene": "UniProtKB:P02778",
  "gene_name": "C-X-C motif chemokine 10",
  "term_id": "GO:0071222"
}